diaminopropionate ammonia-lyase activity [GO:0008838] (molecular function) Also known as: 2,3-diaminopropionate ammonia-lyase (adding H2O; pyruvate-forming), 2,3-diaminopropionate ammonia-lyase activity, alpha,beta-diaminopropionate ammonia-lyase activity, diaminopropionatase activity Definition: Catalysis of the reaction: 2,3-diaminopropionate + H2O = pyruvate + 2 NH3. Relationships: is a type of ammonia-lyase activity [GO:0016841] Sources: EC:4.3.1.15